{
  "term_label": "mitochondrial inner membrane",
  "gene_name": "ATP synthase subunit epsilon, mitochondrial",
  "gene": "UniProtKB:P56381",
  "gene_symbol": "ATP5F1E",
  "term_id": "GO:0005743"
}